{
  "gene_name": "Protein S100-Z",
  "term_id": "GO:0048306",
  "term_label": "calcium-dependent protein binding",
  "gene": "UniProtKB:Q8WXG8",
  "gene_symbol": "S100Z"
}